{
  "gene_name": "Serine_threonine-protein kinase Chk1",
  "term_label": "Unknown cellular component",
  "gene_symbol": "CHEK1",
  "term_id": "UNKNOWN:0003",
  "gene": "UniProtKB:O14757"
}